{
  "term_label": "T cell receptor signaling pathway",
  "gene": "UniProtKB:Q06187",
  "gene_name": "Tyrosine-protein kinase BTK",
  "term_id": "GO:0050852",
  "gene_symbol": "BTK"
}